{
  "gene_symbol": "KLK8",
  "gene_name": "Kallikrein-8",
  "gene": "UniProtKB:O60259",
  "term_id": "GO:0004252",
  "term_label": "serine-type endopeptidase activity"
}